{
  "term_label": "acetylcholine receptor signaling pathway",
  "gene_name": "Neuronal acetylcholine receptor subunit alpha-6",
  "gene_symbol": "CHRNA6",
  "gene": "UniProtKB:Q15825",
  "term_id": "GO:0095500"
}